{
  "gene": "UniProtKB:Q96NT1",
  "term_id": "UNKNOWN:0003",
  "gene_symbol": "NAP1L5",
  "term_label": "Unknown cellular component",
  "gene_name": "Nucleosome assembly protein 1-like 5"
}